{
  "term_id": "GO:0015631",
  "gene": "UniProtKB:Q14679",
  "term_label": "tubulin binding",
  "gene_symbol": "TTLL4",
  "gene_name": "Tubulin monoglutamylase TTLL4"
}